{
  "gene_name": "Protein UXT",
  "term_label": "Unknown biological process",
  "gene": "UniProtKB:Q9UBK9",
  "gene_symbol": "UXT",
  "term_id": "UNKNOWN:0002"
}